{
  "gene_symbol": "CCSAP",
  "term_label": "ciliary transition zone",
  "term_id": "GO:0035869",
  "gene_name": "Centriole, cilia and spindle-associated protein",
  "gene": "UniProtKB:Q6IQ19"
}